sulfate transmembrane transporter activity [GO:0015116] (molecular function) Definition: Enables the transfer of sulfate ions, SO4(2-), from one side of a membrane to the other. Sources: GOC:ai Also known as: sulphate transporter activity, sulfate permease activity Relationships: is a type of sulfur compound transmembrane transporter activity [GO:1901682]; is part of sulfate transmembrane transport [GO:1902358] Subtypes: GO:0005340, secondary active sulfate transmembrane transporter activity [GO:0008271], ABC-type sulfate transporter activity [GO:0015419]